{
  "term_id": "GO:0005739",
  "gene_name": "ATPase family AAA domain-containing protein 3C",
  "gene": "UniProtKB:Q5T2N8",
  "term_label": "mitochondrion",
  "gene_symbol": "ATAD3C"
}